starts during [RO:0002091] (external)